{
  "term_label": "extracellular matrix",
  "gene_name": "Phosphatidylinositol-glycan-specific phospholipase D",
  "gene": "UniProtKB:P80108",
  "term_id": "GO:0031012",
  "gene_symbol": "GPLD1"
}